negative regulation of G2/M transition of mitotic cell cycle [GO:0010972] (biological process) Relationships: is a type of GO:0010389; is a type of negative regulation of mitotic cell cycle phase transition [GO:1901991]; is a type of negative regulation of cell cycle G2/M phase transition [GO:1902750]; negatively regulates G2/M transition of mitotic cell cycle [GO:0000086] Sources: GOC:mtg_cell_cycle Subtypes: mitotic G2 cell size control checkpoint signaling [GO:0031569], GO:0044818, GO:0044878 Definition: Any signaling pathway that decreases or inhibits the activity of a cell cycle cyclin-dependent protein kinase to modulate the switch from G2 phase to M phase of the mitotic cell cycle. Also known as: negative regulation of mitotic entry